2-dehydropantolactone reductase (A-specific) activity [GO:0047011] (MF) Relationships: is_a GO:0036441 Also known as: 2-ketopantoyl lactone reductase activity, 2-oxopantoyl lactone reductase, ketopantoyl lactone reductase activity, (R)-pantolactone:NADP+ oxidoreductase (A-specific), 2-dehydropantoyl-lactone reductase (A-specific) activity Sources: EC:1.1.1.168, MetaCyc:1.1.1.168-RXN Definition: Catalysis of the reaction: (R)-pantolactone + NADP+ = 2-dehydropantolactone + NADPH + H+. The reaction is A-specific (i.e. the pro-R hydrogen is transferred from the 4-position of reduced nicotinamide cofactor) with respect to NADP+.